{
  "gene_symbol": "MRPL11",
  "term_id": "GO:0070180",
  "gene_name": "Large ribosomal subunit protein uL11m",
  "term_label": "large ribosomal subunit rRNA binding",
  "gene": "UniProtKB:Q9Y3B7"
}